antigen processing and presentation initiated by receptor mediated uptake of antigen [GO:0002745] (biological process) Subtypes: antigen processing and presentation initiated by pattern recognition receptor mediated uptake of antigen [GO:0002748], antigen processing and presentation following receptor mediated endocytosis [GO:0002751] Definition: Antigen processing and presentation which is initiated by uptake of antigen bound to a cell surface receptor. Sources: GOC:add, ISBN:0781735149 Relationships: is_a antigen processing and presentation [GO:0019882]